{
  "term_id": "GO:0006867",
  "term_label": "asparagine transport",
  "gene_name": "Sodium-coupled neutral amino acid transporter 3",
  "gene_symbol": "SLC38A3",
  "gene": "UniProtKB:Q99624"
}